{
  "gene_symbol": "NIPAL3",
  "term_label": "magnesium ion transport",
  "gene": "UniProtKB:Q6P499",
  "gene_name": "NIPA-like protein 3",
  "term_id": "GO:0015693"
}